molecular template activity [GO:0140489] (molecular function) Relationships: is a type of molecular_function [GO:0003674] Subtypes: DNA template activity [GO:0000497], GO:0140490 Definition: The action of a molecule that provides a shape or a sequence mimicking or complementary to the final product, providing template for copying the original molecule's shape or sequence. Sources: GOC:pg